proteasomal ubiquitin-independent protein catabolic process [GO:0010499] (biological process) Relationships: is a type of proteasomal protein catabolic process [GO:0010498] Definition: The chemical reactions and pathways resulting in the breakdown of a protein or peptide by hydrolysis of its peptide bonds that is mediated by the proteasome but do not involve ubiquitin. Sources: GOC:tb